{
  "gene_symbol": "P2RY11",
  "gene_name": "P2Y purinoceptor 11",
  "gene": "UniProtKB:Q96G91",
  "term_id": "GO:0030594",
  "term_label": "neurotransmitter receptor activity"
}